resveratrol 3,5-O-dimethyltransferase activity [GO:0102303] (molecular function) Definition: Catalysis of the reaction: 2 S-adenosyl-L-methionine + trans-resveratrol = 2 S-adenosyl-L-homocysteine + pterostilbene + 2 H+. Relationships: is_a methyltransferase activity [GO:0008168] Sources: EC:2.1.1.240, GOC:pz